{
  "term_label": "Unknown cellular component",
  "gene": "UniProtKB:A1A5C7",
  "gene_name": "Solute carrier family 22 member 23",
  "term_id": "UNKNOWN:0003",
  "gene_symbol": "SLC22A23"
}